NK T cell activation [GO:0051132] (biological process) Definition: The change in morphology and behavior of a mature or immature natural killer T cell resulting from exposure to a mitogen, cytokine, chemokine, cellular ligand, or an antigen for which it is specific. Subtypes: NK T cell proliferation [GO:0001866], NK T cell activation involved in immune response [GO:0002288] Note: Note that NK T cells are a distinct lineage of T cells expressing natural killer cell markers and having T cell receptors characterized by the usage of a restricted repertoire of variable region gene segments. Also known as: NK T lymphocyte activation, NK T-cell activation, NK T-lymphocyte activation, NKT cell activation, NT cell activation, natural T cell activation, natural killer T cell activation Regulation: regulated by regulation of NK T cell activation [GO:0051133]; negatively regulated by negative regulation of NK T cell activation [GO:0051134]; positively regulated by positive regulation of NK T cell activation [GO:0051135] Relationships: is a type of alpha-beta T cell activation [GO:0046631] References: PMID:12154375, PMID:9133426 Sources: ISBN:0781735149